intracellular water homeostasis [GO:0009992] (biological process) Relationships: is a type of cell volume homeostasis [GO:0006884]; is a type of intracellular chemical homeostasis [GO:0055082] Also known as: cellular water homeostasis, cellular osmoregulation Definition: A homeostatic process involved in the maintenance of a steady state level of water within a cell. Sources: GOC:dph, GOC:tb